{
  "term_label": "SNARE complex",
  "gene_name": "Vesicle transport protein USE1",
  "term_id": "GO:0031201",
  "gene_symbol": "USE1",
  "gene": "UniProtKB:Q9NZ43"
}